ganglion morphogenesis [GO:0061552] (biological process) Definition: The process in which the anatomical structures of ganglion are generated and organized. Subtypes: GO:0061559, dorsal root ganglion morphogenesis [GO:1904835] Relationships: is a type of GO:0048729; is part of ganglion development [GO:0061548] Also known as: ganglia morphogenesis Sources: GOC:dph